positive regulation of negative chemotaxis [GO:0050924] (biological process) Subtypes: GO:0050929 Relationships: is a type of GO:0050921; is a type of regulation of negative chemotaxis [GO:0050923]; positively regulates negative chemotaxis [GO:0050919] Also known as: up regulation of negative chemotaxis, up-regulation of negative chemotaxis, upregulation of negative chemotaxis, activation of negative chemotaxis, stimulation of negative chemotaxis Sources: GOC:ai Definition: Any process that activates or increases the frequency, rate or extent of the directed movement of a motile cell or organism towards a lower concentration in a concentration gradient of a specific chemical.